{
  "gene_symbol": "GPR37",
  "gene_name": "Prosaposin receptor GPR37",
  "term_id": "GO:0007193",
  "term_label": "adenylate cyclase-inhibiting G protein-coupled receptor signaling pathway",
  "gene": "UniProtKB:O15354"
}